{
  "gene": "UniProtKB:Q9BYX7",
  "gene_symbol": "POTEKP",
  "term_label": "axonogenesis",
  "gene_name": "Putative beta-actin-like protein 3",
  "term_id": "GO:0007409"
}